guanyl-nucleotide exchange factor adaptor activity [GO:0005091] (molecular function) Definition: The binding activity of a molecule that brings together a guanyl-nucleotide exchange factor and one or more other proteins, permitting them to function in a coordinated way. Sources: GOC:mtg_MIT_16mar07, GOC:vw Relationships: is a type of GO:0030674; is a type of GTPase regulator activity [GO:0030695]